telomere-nuclear envelope anchor activity [GO:0140473] (molecular function) Relationships: is a type of protein-membrane adaptor activity [GO:0043495] Definition: The binding activity of a molecule that brings together the telomeric region of a chromosome and the inner nuclear membrane by interacting with both the telomere and the nuclear membrane, in order to establish and maintain the telomeric location. References: PMID:31635174 Also known as: nuclear envelope-telomere anchor activity, telomere-nuclear envelope anchoring activity